{
  "gene": "UniProtKB:Q00169",
  "gene_symbol": "PITPNA",
  "gene_name": "Phosphatidylinositol transfer protein alpha isoform",
  "term_label": "phosphatidylcholine binding",
  "term_id": "GO:0031210"
}